{
  "gene": "UniProtKB:Q5TH69",
  "gene_symbol": "ARFGEF3",
  "gene_name": "Brefeldin A-inhibited guanine nucleotide-exchange protein 3",
  "term_label": "vesicle-mediated transport",
  "term_id": "GO:0016192"
}